cellular response to UV-A [GO:0071492] (biological process) Sources: GOC:mah Also known as: cellular response to UV-A light stimulus, cellular response to UV-A radiation stimulus, cellular response to UVA light stimulus, cellular response to UVA radiation stimulus Definition: Any process that results in a change in state or activity of a cell (in terms of movement, secretion, enzyme production, gene expression, etc.) as a result of a UV-A radiation stimulus. UV-A radiation (UV-A light) spans the wavelengths 315 to 400 nm. Relationships: is a type of GO:0034644; is a type of response to UV-A [GO:0070141]